allantois development [GO:1905069] (biological process) Definition: The process whose specific outcome is the progression of an allantois over time, from its formation to the mature structure. References: PMID:17440924, PMID:21470579 Sources: GOC:TermGenie, GO_REF:0000094 Also known as: allantoic bud development Relationships: is a type of extraembryonic membrane development [GO:1903867]